{
  "term_id": "GO:0005886",
  "gene": "UniProtKB:Q8NGE5",
  "gene_symbol": "OR10A7",
  "term_label": "plasma membrane",
  "gene_name": "Olfactory receptor 10A7"
}